{
  "term_label": "positive regulation of autophagy",
  "gene": "UniProtKB:P49840",
  "term_id": "GO:0010508",
  "gene_name": "Glycogen synthase kinase-3 alpha",
  "gene_symbol": "GSK3A"
}